{
  "gene_symbol": "ALDH9A1",
  "term_id": "GO:0019145",
  "gene": "UniProtKB:P49189",
  "gene_name": "4-trimethylaminobutyraldehyde dehydrogenase",
  "term_label": "aminobutyraldehyde dehydrogenase (NAD+) activity"
}